{
  "gene_name": "Protein YIF1B",
  "gene_symbol": "YIF1B",
  "term_id": "GO:0005789",
  "gene": "UniProtKB:Q5BJH7",
  "term_label": "endoplasmic reticulum membrane"
}